{
  "gene": "UniProtKB:Q9Y6K8",
  "gene_name": "Adenylate kinase isoenzyme 5",
  "term_label": "nucleoside diphosphate kinase activity",
  "term_id": "GO:0004550",
  "gene_symbol": "AK5"
}